UTP:glucose-1-phosphate uridylyltransferase regulator activity [GO:0043763] (MF) Sources: GOC:jl Relationships: is a type of enzyme regulator activity [GO:0030234]; regulates UTP:glucose-1-phosphate uridylyltransferase activity [GO:0003983] Definition: Binds to and modulates the activity of UTP:glucose-1-phosphate uridylyltransferase. Also known as: UDP-glucose diphosphorylase regulator activity, UDP-glucose pyrophosphorylase regulator activity, glucose-1-phosphate uridylyltransferase regulator activity